{
  "gene_name": "Alsin",
  "term_label": "endosomal transport",
  "gene_symbol": "ALS2",
  "term_id": "GO:0016197",
  "gene": "UniProtKB:Q96Q42"
}